positive regulation of SREBP signaling pathway in response to decreased oxygen levels [GO:0038176] (biological process) Relationships: is a type of GO:2000640; is part of GO:0036294 Definition: Any process that activates or increases the frequency, rate or extent of the SREBP signaling pathway in response to a decrease in oxygen levels. References: PMID:22017871 Sources: GOC:al Also known as: positive regulation of SREBP-mediated signaling pathway in response to decreased oxygen levels, positive regulation of SREBP-mediated signaling pathway in absence of oxygen